{
  "gene_symbol": "PLEKHD1",
  "term_id": "UNKNOWN:0002",
  "gene_name": "Pleckstrin homology domain-containing family D member 1",
  "term_label": "Unknown biological process",
  "gene": "UniProtKB:A6NEE1"
}